{
  "gene_name": "Ribosome biogenesis regulatory protein homolog",
  "gene": "UniProtKB:Q15050",
  "gene_symbol": "RRS1",
  "term_id": "GO:0030687",
  "term_label": "preribosome, large subunit precursor"
}